{
  "gene_symbol": "NSUN3",
  "term_id": "GO:0008168",
  "gene_name": "tRNA (cytosine(34)-C(5))-methyltransferase, mitochondrial",
  "term_label": "methyltransferase activity",
  "gene": "UniProtKB:Q9H649"
}